{
  "term_id": "UNKNOWN:0002",
  "gene_name": "Secretoglobin family 3A member 2",
  "gene_symbol": "SCGB3A2",
  "gene": "UniProtKB:Q96PL1",
  "term_label": "Unknown biological process"
}